{
  "gene": "UniProtKB:Q9NPC8",
  "gene_name": "Homeobox protein SIX2",
  "term_id": "GO:0000978",
  "term_label": "RNA polymerase II cis-regulatory region sequence-specific DNA binding",
  "gene_symbol": "SIX2"
}